{
  "term_label": "Unknown biological process",
  "term_id": "UNKNOWN:0002",
  "gene_symbol": "KRTAP19-1",
  "gene_name": "Keratin-associated protein 19-1",
  "gene": "UniProtKB:Q8IUB9"
}